{
  "gene_name": "Ubiquitin-fold modifier-conjugating enzyme 1",
  "term_id": "GO:0034976",
  "gene": "UniProtKB:Q9Y3C8",
  "gene_symbol": "UFC1",
  "term_label": "response to endoplasmic reticulum stress"
}